{
  "gene": "UniProtKB:P52741",
  "gene_symbol": "ZNF134",
  "term_label": "DNA-binding transcription repressor activity, RNA polymerase II-specific",
  "term_id": "GO:0001227",
  "gene_name": "Zinc finger protein 134"
}